{
  "gene": "UniProtKB:A0A087WSY4",
  "term_label": "antigen binding",
  "gene_symbol": "IGHV4-30-2",
  "term_id": "GO:0003823",
  "gene_name": "Immunoglobulin heavy variable 4-30-2"
}